{
  "term_id": "GO:0007399",
  "gene_name": "Tyrosine-protein kinase receptor TYRO3",
  "gene_symbol": "TYRO3",
  "gene": "UniProtKB:Q06418",
  "term_label": "nervous system development"
}